ribonuclease [poly-(U)-specific] activity [GO:0033895] (MF) Also known as: ribonuclease (uracil-specific) activity, uracil-specific RNase activity, uracil-specific endoribonuclease activity Definition: Catalysis of the endonucleolytic cleavage of poly(U) to fragments terminated by 3'-hydroxy and 5'-phosphate groups. Sources: EC:3.1.26.9 Relationships: is a type of RNA endonuclease activity producing 5'-phosphomonoesters, hydrolytic mechanism [GO:0016891]